{
  "gene_name": "Copine-8",
  "term_id": "GO:0071277",
  "gene": "UniProtKB:Q86YQ8",
  "term_label": "cellular response to calcium ion",
  "gene_symbol": "CPNE8"
}